{
  "term_label": "signal transduction",
  "gene_name": "Receptor-type tyrosine-protein phosphatase gamma",
  "gene": "UniProtKB:P23470",
  "term_id": "GO:0007165",
  "gene_symbol": "PTPRG"
}